response to tert-butyl hydroperoxide [GO:0072735] (biological process) Subtypes: cellular response to tert-butyl hydroperoxide [GO:0072736] Definition: Any process that results in a change in state or activity of a cell or an organism (in terms of movement, secretion, enzyme production, gene expression, etc.) as a result of a tert-butyl hydroperoxide (t-BOOH) stimulus. Relationships: is_a GO:0033195 Also known as: response to 2-methyl-prop-2-yl-hydroperoxide, response to t-BOOH Sources: GOC:mah